positive regulation of tolerance induction [GO:0002645] (biological process) Also known as: up regulation of tolerance induction, up-regulation of tolerance induction, upregulation of tolerance induction, activation of tolerance induction, stimulation of tolerance induction Subtypes: GO:0002648, positive regulation of tolerance induction to self antigen [GO:0002651], positive regulation of tolerance induction dependent upon immune response [GO:0002654], positive regulation of B cell tolerance induction [GO:0002663], positive regulation of T cell tolerance induction [GO:0002666], positive regulation of natural killer cell tolerance induction [GO:0002873], positive regulation of lymphocyte anergy [GO:0002913], GO:0010933 Sources: GOC:add Definition: Any process that activates or increases the frequency, rate, or extent of tolerance induction. Relationships: is a type of regulation of tolerance induction [GO:0002643]; is a type of positive regulation of immune system process [GO:0002684]; is a type of positive regulation of multicellular organismal process [GO:0051240]; positively regulates tolerance induction [GO:0002507]